{
  "term_id": "GO:0070588",
  "term_label": "calcium ion transmembrane transport",
  "gene_name": "Sodium_potassium_calcium exchanger 4",
  "gene_symbol": "SLC24A4",
  "gene": "UniProtKB:Q8NFF2"
}